{
  "gene": "UniProtKB:P0CJ77",
  "gene_symbol": "MTRNR2L10",
  "gene_name": "Humanin-like 10",
  "term_id": "GO:1900118",
  "term_label": "negative regulation of execution phase of apoptosis"
}